{
  "term_label": "neuromuscular junction",
  "term_id": "GO:0031594",
  "gene": "UniProtKB:O95473",
  "gene_name": "Synaptogyrin-4",
  "gene_symbol": "SYNGR4"
}